{
  "term_label": "synaptic vesicle fusion to presynaptic active zone membrane",
  "gene": "UniProtKB:O95721",
  "gene_name": "Synaptosomal-associated protein 29",
  "term_id": "GO:0031629",
  "gene_symbol": "SNAP29"
}